U5 snRNA binding [GO:0030623] (molecular function) Definition: Binding to a U5 small nuclear RNA (U5 snRNA). Sources: GOC:jl Relationships: is a type of snRNA binding [GO:0017069]